{
  "term_label": "cytoplasm",
  "gene_symbol": "TNPO3",
  "term_id": "GO:0005737",
  "gene_name": "Transportin-3",
  "gene": "UniProtKB:Q9Y5L0"
}